pairing center [GO:0036224] (cellular component) Also known as: homolog recognition region Relationships: is a type of GO:0110165; is part of condensed nuclear chromosome [GO:0000794] References: PMID:18597662 Sources: GOC:kmv Definition: A special chromosome region located towards one end of a chromosome that contains dispersed copies of short, repetitive DNA sequences and functions as a cis-acting element essential for presynaptic homologous chromosome pairing and chromosome-nuclear envelope attachment.